xylose isomerase activity [GO:0009045] (molecular function) Definition: Catalysis of the reaction: alpha-D-xylose = alpha-D-xylulofuranose. Sources: RHEA:22816 Relationships: is a type of GO:0016861 Also known as: D-xylose aldose-ketose-isomerase activity, D-xylose isomerase activity, D-xylose ketoisomerase activity, D-xylose ketol-isomerase activity